{
  "term_id": "UNKNOWN:0001",
  "term_label": "Unknown molecular function",
  "gene_symbol": "PALM2AKAP2",
  "gene_name": "PALM2 and AKAP2 fusion",
  "gene": "UniProtKB:C9JA33"
}